{
  "gene_name": "Creatine kinase B-type",
  "gene": "UniProtKB:P12277",
  "gene_symbol": "CKB",
  "term_id": "GO:0005615",
  "term_label": "extracellular space"
}